{
  "gene_symbol": "CLSTN1",
  "gene_name": "Calsyntenin-1",
  "gene": "UniProtKB:O94985",
  "term_label": "positive regulation of synapse assembly",
  "term_id": "GO:0051965"
}